{
  "term_label": "Unknown cellular component",
  "gene_symbol": "C19orf18",
  "term_id": "UNKNOWN:0003",
  "gene": "UniProtKB:Q8NEA5",
  "gene_name": "Uncharacterized protein C19orf18"
}